{
  "term_id": "GO:0140375",
  "term_label": "immune receptor activity",
  "gene_name": "Killer cell immunoglobulin-like receptor 2DS3",
  "gene": "UniProtKB:Q14952",
  "gene_symbol": "KIR2DS3"
}